L-lysine transmembrane import into vacuole [GO:0090517] (biological process) Definition: The directed movement of L-lysine into the vacuole across the vacuolar membrane. Also known as: lysine transmembrane import into vacuole, vacuolar lysine import Subtypes: GO:1901482 Relationships: is a type of lysine transport [GO:0015819]; is a type of GO:0034490; is a type of L-lysine transmembrane transport [GO:1903401] Sources: GOC:al